{
  "term_label": "transcription coactivator activity",
  "term_id": "GO:0003713",
  "gene_name": "CREB-regulated transcription coactivator 2",
  "gene_symbol": "CRTC2",
  "gene": "UniProtKB:Q53ET0"
}